lung alveolus development [GO:0048286] (biological process) Definition: The process whose specific outcome is the progression of the alveolus over time, from its formation to the mature structure. The alveolus is a sac for holding air in the lungs; formed by the terminal dilation of air passageways. References: PMID:9751757 Sources: GOC:mtg_lung Also known as: alveolarization, alveologenesis Relationships: is_a anatomical structure development [GO:0048856]; is part of lung development [GO:0030324] Regulation: regulated by regulation of lung alveolus development [GO:1904653]; RO_0002212 by negative regulation of lung alveolus development [GO:1904654]; positively regulated by positive regulation of lung alveolus development [GO:1904655]